{
  "gene_name": "Zinc finger protein 699",
  "gene": "UniProtKB:Q32M78",
  "term_id": "GO:0000981",
  "term_label": "DNA-binding transcription factor activity, RNA polymerase II-specific",
  "gene_symbol": "ZNF699"
}